{
  "gene_name": "Serpin B4",
  "term_id": "GO:0005615",
  "gene_symbol": "SERPINB4",
  "gene": "UniProtKB:P48594",
  "term_label": "extracellular space"
}